{
  "gene_name": "Exonuclease 1",
  "gene_symbol": "EXO1",
  "term_id": "GO:0005634",
  "gene": "UniProtKB:Q9UQ84",
  "term_label": "nucleus"
}